{
  "gene": "UniProtKB:P31249",
  "term_id": "GO:0000981",
  "term_label": "DNA-binding transcription factor activity, RNA polymerase II-specific",
  "gene_name": "Homeobox protein Hox-D3",
  "gene_symbol": "HOXD3"
}